blood vessel maturation [GO:0001955] (biological process) Relationships: is a type of anatomical structure maturation [GO:0071695]; is part of blood vessel development [GO:0001568] Sources: GOC:dph Definition: A developmental process, independent of morphogenetic (shape) change, that is required for a blood vessel to attain its fully functional state.